{
  "term_id": "GO:0060397",
  "gene_symbol": "JAK1",
  "gene_name": "Tyrosine-protein kinase JAK1",
  "term_label": "growth hormone receptor signaling pathway via JAK-STAT",
  "gene": "UniProtKB:P23458"
}